{
  "gene_symbol": "NIPBL",
  "gene": "UniProtKB:Q6KC79",
  "term_id": "GO:0071169",
  "term_label": "establishment of protein localization to chromatin",
  "gene_name": "Nipped-B-like protein"
}